{
  "gene_symbol": "CC2D2B",
  "gene_name": "Protein CC2D2B",
  "gene": "UniProtKB:Q6DHV5",
  "term_id": "GO:0035869",
  "term_label": "ciliary transition zone"
}